{
  "gene": "UniProtKB:Q6ZMN7",
  "gene_symbol": "PDZRN4",
  "gene_name": "PDZ domain-containing RING finger protein 4",
  "term_label": "Unknown biological process",
  "term_id": "UNKNOWN:0002"
}